{
  "gene_symbol": "CCDC86",
  "gene_name": "Coiled-coil domain-containing protein 86",
  "term_id": "UNKNOWN:0002",
  "term_label": "Unknown biological process",
  "gene": "UniProtKB:Q9H6F5"
}